{
  "gene_symbol": "SGSH",
  "gene": "UniProtKB:P51688",
  "term_id": "GO:0030200",
  "gene_name": "N-sulphoglucosamine sulphohydrolase",
  "term_label": "heparan sulfate proteoglycan catabolic process"
}